{
  "term_label": "endosomal transport",
  "term_id": "GO:0016197",
  "gene_name": "Neuronal vesicle trafficking-associated protein 2",
  "gene": "UniProtKB:Q9Y328",
  "gene_symbol": "NSG2"
}